host cell cytoplasmic vesicle [GO:0044161] (cellular component) Subtypes: host cell synaptic vesicle [GO:0098584] Definition: A vesicle formed of membrane or protein, found in the cytoplasm of a host cell. Relationships: is a type of host intracellular membrane-bounded organelle [GO:0033648]; is a type of host cell cytoplasm part [GO:0033655] Sources: GOC:rph